purine deoxyribonucleoside salvage [GO:0043098] (biological process) Relationships: is a type of purine-containing compound salvage [GO:0043101]; is a type of nucleoside salvage [GO:0043174]; is a type of purine deoxyribonucleoside biosynthetic process [GO:0046123] Definition: Any process which produces a purine deoxyribonucleoside from derivatives of it, without de novo synthesis. Sources: GOC:jl Subtypes: deoxyguanosine salvage [GO:0006180], GO:0006191